{
  "gene": "UniProtKB:Q9NX57",
  "term_id": "GO:0030139",
  "gene_symbol": "RAB20",
  "gene_name": "Ras-related protein Rab-20",
  "term_label": "endocytic vesicle"
}